regulation of dolichyl monophosphate biosynthetic process [GO:0010794] (biological process) Also known as: regulation of dolichol biosynthetic process Definition: Any process that modulates the frequency, rate or extent of dolichol biosynthesis. Dolichol biosynthesis consists of the chemical reactions and pathways resulting in the formation of dolichols, any 2,3-dihydropolyprenol derived from four or more linked isoprene units. Sources: GOC:dph, GOC:tb Relationships: is a type of regulation of phospholipid biosynthetic process [GO:0071071]; regulates GO:0043048